{
  "term_label": "Unknown biological process",
  "gene_symbol": "DGCR6L",
  "gene_name": "Protein DGCR6L",
  "gene": "UniProtKB:Q9BY27",
  "term_id": "UNKNOWN:0002"
}